{
  "term_label": "ubiquitin protein ligase activity",
  "gene_name": "Putative HERC2-like protein 3",
  "gene_symbol": "HERC2P3",
  "term_id": "GO:0061630",
  "gene": "UniProtKB:Q9BVR0"
}